{
  "term_id": "GO:0005615",
  "gene_symbol": "PLAU",
  "gene": "UniProtKB:P00749",
  "gene_name": "Urokinase-type plasminogen activator",
  "term_label": "extracellular space"
}